{
  "gene": "UniProtKB:Q6RW13",
  "gene_symbol": "AGTRAP",
  "term_id": "GO:0008217",
  "term_label": "regulation of blood pressure",
  "gene_name": "Type-1 angiotensin II receptor-associated protein"
}